fungal-type cell wall [GO:0009277] (cellular component) Definition: A rigid yet dynamic structure surrounding the plasma membrane that affords protection from stresses and contributes to cell morphogenesis, consisting of extensively cross-linked glycoproteins and carbohydrates. The glycoproteins may be modified with N- or O-linked carbohydrates, or glycosylphosphatidylinositol (GPI) anchors; the polysaccharides are primarily branched glucans, including beta-linked and alpha-linked glucans, and may also include chitin and other carbohydrate polymers, but not cellulose or pectin. Enzymes involved in cell wall biosynthesis are also found in the cell wall. Note that some forms of fungi develop a capsule outside of the cell wall under certain circumstances; this is considered a separate structure. References: PMID:11283274, PMID:16927300, PMID:3319422 Sources: GOC:mcc, GOC:mtg_sensu, ISBN:3540601864 Also known as: chitin- and beta-glucan-containing cell wall, beta-glucan-containing cell wall, chitin-containing cell wall Relationships: is a type of cell wall [GO:0005618] Subtypes: ascospore wall [GO:0005619], GO:0030445, hyphal cell wall [GO:0030446]